{
  "term_label": "cytoplasm",
  "gene_name": "Kelch-like protein 30",
  "gene": "UniProtKB:Q0D2K2",
  "term_id": "GO:0005737",
  "gene_symbol": "KLHL30"
}